{
  "term_id": "GO:0036503",
  "term_label": "ERAD pathway",
  "gene_symbol": "PSMC6",
  "gene": "UniProtKB:P62333",
  "gene_name": "26S proteasome regulatory subunit 10B"
}